{
  "gene_symbol": "C2CD2L",
  "term_id": "GO:0035091",
  "gene": "UniProtKB:O14523",
  "term_label": "phosphatidylinositol binding",
  "gene_name": "Phospholipid transfer protein C2CD2L"
}